{
  "gene_name": "A-kinase anchor protein 17A",
  "term_label": "nuclear speck",
  "gene": "UniProtKB:Q02040",
  "term_id": "GO:0016607",
  "gene_symbol": "AKAP17A"
}